{
  "term_id": "UNKNOWN:0003",
  "term_label": "Unknown cellular component",
  "gene": "UniProtKB:Q9HB75",
  "gene_symbol": "PIDD1",
  "gene_name": "p53-induced death domain-containing protein 1"
}